positive regulation of monocyte chemotaxis [GO:0090026] (biological process) Relationships: is a type of positive regulation of leukocyte chemotaxis [GO:0002690]; is a type of positive regulation of mononuclear cell migration [GO:0071677]; is a type of regulation of monocyte chemotaxis [GO:0090025]; positively regulates monocyte chemotaxis [GO:0002548] Definition: Any process that increases the frequency, rate, or extent of monocyte chemotaxis. Sources: GOC:dph, GOC:tb